{
  "term_label": "translation activator activity",
  "gene_name": "Deleted in azoospermia protein 4",
  "gene": "UniProtKB:Q86SG3",
  "gene_symbol": "DAZ4",
  "term_id": "GO:0008494"
}